{
  "gene_symbol": "KIF3B",
  "term_label": "microtubule binding",
  "term_id": "GO:0008017",
  "gene": "UniProtKB:O15066",
  "gene_name": "Kinesin-like protein KIF3B"
}